{
  "gene_symbol": "GSTM4",
  "term_label": "Unknown cellular component",
  "term_id": "UNKNOWN:0003",
  "gene_name": "Glutathione S-transferase Mu 4",
  "gene": "UniProtKB:Q03013"
}